cell chemotaxis [GO:0060326] (biological process) Subtypes: leukocyte chemotaxis [GO:0030595], GO:0035232, germ cell repulsion [GO:0035233], GO:0035700, cell chemotaxis to fibroblast growth factor [GO:0035766], endothelial cell chemotaxis [GO:0035767], muscle cell chemotaxis toward tendon cell [GO:0036061], cell chemotaxis involved in Malpighian tubule morphogenesis [GO:0061352], GO:0061583, cell chemotaxis to angiotensin [GO:0071434], GO:0071670, cell chemotaxis to vascular endothelial growth factor [GO:0090667], GO:1990751, GO:1990956 Relationships: is a type of chemotaxis [GO:0006935]; is a type of cell migration [GO:0016477]; is part of cellular response to chemical stimulus [GO:0070887] Sources: GOC:dph Definition: The directed movement of a motile cell guided by a specific chemical concentration gradient. Movement may be towards a higher concentration (positive chemotaxis) or towards a lower concentration (negative chemotaxis).